{
  "gene_symbol": "IRX6",
  "term_label": "RNA polymerase II cis-regulatory region sequence-specific DNA binding",
  "gene_name": "Iroquois-class homeodomain protein IRX-6",
  "term_id": "GO:0000978",
  "gene": "UniProtKB:P78412"
}